{
  "gene_symbol": "SLC17A9",
  "term_label": "Unknown molecular function",
  "gene": "UniProtKB:Q9BYT1",
  "term_id": "UNKNOWN:0001",
  "gene_name": "Voltage-gated purine nucleotide uniporter SLC17A9"
}